atrioventricular canal development [GO:0036302] (biological process) Definition: The progression of the atrioventricular canal over time, from its formation to the mature structure. The atrioventricular canal is the part of the heart connecting the atrium to the cardiac ventricle. References: PMID:14701881 Sources: GOC:BHF, GOC:gr, UBERON:0002087, ZFA:0001315 Relationships: is a type of anatomical structure development [GO:0048856]; is part of heart development [GO:0007507]